{
  "gene_symbol": "OXR1",
  "term_label": "Unknown molecular function",
  "term_id": "UNKNOWN:0001",
  "gene_name": "Oxidation resistance protein 1",
  "gene": "UniProtKB:Q8N573"
}